ceramide transfer activity [GO:0120017] (molecular function) References: PMID:20823909, PMID:24220498, PMID:25797198 Sources: GOC:krc Relationships: is a type of GO:0120016; has part GO:0097001 Also known as: ceramide transporter activity, ceramide carrier activity, intermembrane ceramide transfer activity Subtypes: GO:0140340, ceramide 1-phosphate transfer activity [GO:1902388] Definition: Removes a ceramide from a membrane or a monolayer lipid particle, transports it through the aqueous phase while protected in a hydrophobic pocket, and brings it to an acceptor membrane or lipid particle.